aurone biosynthetic process [GO:0051551] (biological process) Definition: The chemical reactions and pathways resulting in the formation of aurones, a series of yellow plant pigments. References: PMID:20035037 Sources: GOC:ai Relationships: is_a flavonoid biosynthetic process [GO:0009813]; is a type of GO:0042181; is a type of GO:0046148 Also known as: benzalcoumaran-3-one biosynthesis, benzalcoumaran-3-one biosynthetic process